{
  "gene_symbol": "FCGR2B",
  "term_id": "GO:0019770",
  "gene_name": "Low affinity immunoglobulin gamma Fc region receptor II-b",
  "gene": "UniProtKB:P31994",
  "term_label": "IgG receptor activity"
}